{
  "gene": "UniProtKB:Q8WTR4",
  "term_label": "plasma membrane",
  "gene_symbol": "GDPD5",
  "term_id": "GO:0005886",
  "gene_name": "Glycerophosphodiester phosphodiesterase domain-containing protein 5"
}